{
  "term_label": "Unknown cellular component",
  "term_id": "UNKNOWN:0003",
  "gene": "UniProtKB:A6NDE8",
  "gene_symbol": "GAGE12H",
  "gene_name": "G antigen 12H"
}